{
  "gene_symbol": "DUX3",
  "gene": "UniProtKB:Q96PT4",
  "term_id": "GO:0000977",
  "gene_name": "Putative double homeobox protein 3",
  "term_label": "RNA polymerase II transcription regulatory region sequence-specific DNA binding"
}